{
  "term_id": "GO:0005886",
  "gene": "UniProtKB:Q9NYK1",
  "gene_name": "Toll-like receptor 7",
  "term_label": "plasma membrane",
  "gene_symbol": "TLR7"
}